{
  "gene": "UniProtKB:A0A0C4DH32",
  "gene_name": "Immunoglobulin heavy variable 3-20",
  "gene_symbol": "IGHV3-20",
  "term_label": "antigen binding",
  "term_id": "GO:0003823"
}